ferric iron transmembrane transporter activity [GO:0015091] (molecular function) Subtypes: low-affinity ferric iron ion transmembrane transporter activity [GO:0015090], high-affinity ferric iron transmembrane transporter activity [GO:0015092], ABC-type ferric iron transporter activity [GO:0015408] Note: Ferric iron is rarely transported in the free form. Some bacteria have a system in which an outer membrane protein takes iron away from host ferritin or lactoferrin and transport it to a Fe3+ binding protein in the periplasm. The periplasmic protein then delivers the Fe3+ to a transport system located in the cytoplasmic membrane. Consider also GO:0015343 siderophore transmembrane transporter activity. Relationships: is a type of iron ion transmembrane transporter activity [GO:0005381] Definition: Enables the transfer of ferric iron (Fe(III) or Fe3+) ions from one side of a membrane to the other. Sources: ISBN:0198506732